compound eye development [GO:0048749] (biological process) Sources: GOC:jid, GOC:mtg_sensu, Wikipedia:Eye Relationships: is a type of eye development [GO:0001654] Definition: The process whose specific outcome is the progression of the compound eye over time, from its formation to the mature structure. The compound eye is an organ of sight that contains multiple repeating units, often arranged hexagonally. Each unit has its own lens and photoreceptor cell(s) and can generate either a single pixelated image or multiple images, per eye. Also known as: insect-type retina development